{
  "term_id": "UNKNOWN:0001",
  "gene": "UniProtKB:Q9HBL6",
  "term_label": "Unknown molecular function",
  "gene_name": "Leucine-rich repeat and transmembrane domain-containing protein 1",
  "gene_symbol": "LRTM1"
}